{
  "term_id": "GO:0007035",
  "gene_symbol": "ATP6V0D2",
  "gene_name": "V-type proton ATPase subunit d 2",
  "gene": "UniProtKB:Q8N8Y2",
  "term_label": "vacuolar acidification"
}